clathrin coat of trans-Golgi network vesicle [GO:0030130] (cellular component) Sources: GOC:mah Also known as: clathrin coat of TGN vesicle Definition: A clathrin coat found on a vesicle of the trans-Golgi network. Relationships: is a type of clathrin vesicle coat [GO:0030125]; is part of Golgi apparatus [GO:0005794]; is part of GO:0012510